{
  "term_id": "GO:0008017",
  "term_label": "microtubule binding",
  "gene_name": "Fibronectin type III and SPRY domain-containing protein 1",
  "gene": "UniProtKB:Q9BTV5",
  "gene_symbol": "FSD1"
}